{
  "term_label": "xenobiotic metabolic process",
  "gene_name": "Vitamin D 25-hydroxylase",
  "term_id": "GO:0006805",
  "gene_symbol": "CYP2R1",
  "gene": "UniProtKB:Q6VVX0"
}